{
  "term_id": "GO:0035591",
  "gene": "UniProtKB:Q9P2A4",
  "gene_name": "ABI gene family member 3",
  "term_label": "signaling adaptor activity",
  "gene_symbol": "ABI3"
}